{
  "gene_symbol": "PPP1R12A",
  "gene": "UniProtKB:O14974",
  "term_label": "enzyme inhibitor activity",
  "term_id": "GO:0004857",
  "gene_name": "Protein phosphatase 1 regulatory subunit 12A"
}